nicotinamide riboside catabolic process [GO:0006738] (biological process) Definition: The chemical reactions and pathways resulting in the breakdown of nicotinamide riboside, the product of the formation of a glycosidic bond between ribose and nicotinamide. Relationships: is a type of nicotinamide riboside metabolic process [GO:0046495]; is a type of pyridine nucleoside catabolic process [GO:0070638] Sources: ISBN:0198506732 Also known as: N-ribosylnicotinamide catabolic process, nicotinamide riboside breakdown, nicotinamide riboside catabolism, nicotinamide riboside degradation